{
  "gene_symbol": "ARHGEF25",
  "gene_name": "Rho guanine nucleotide exchange factor 25",
  "term_id": "GO:0019898",
  "term_label": "extrinsic component of membrane",
  "gene": "UniProtKB:Q86VW2"
}